SBF transcription complex [GO:0033309] (cellular component) Relationships: is a type of RNA polymerase II transcription regulator complex [GO:0090575] References: PMID:11206552, PMID:15838511, PMID:18160399, PMID:19150335, PMID:7917338 Sources: GOC:mah Also known as: SBF complex Definition: A protein complex that binds to the Swi4/6 cell cycle box (SCB) promoter element, consensus sequence CRCGAAA, and activates transcription during the G1/S transition of the cell cycle. In Saccharomyces, the complex contains a heterodimer of the DNA binding protein Swi4p and the activator Swi6p, and is associated with additional proteins known as Whi5p and Msa1p.